{
  "term_id": "GO:0043023",
  "gene_symbol": "EIF6",
  "gene_name": "Eukaryotic translation initiation factor 6",
  "gene": "UniProtKB:P56537",
  "term_label": "ribosomal large subunit binding"
}